{
  "gene_name": "Fetal and adult testis-expressed transcript protein",
  "term_label": "negative regulation of apoptotic process",
  "gene": "UniProtKB:Q969F0",
  "term_id": "GO:0043066",
  "gene_symbol": "FATE1"
}